{
  "gene": "UniProtKB:Q9UHY8",
  "term_label": "Unknown molecular function",
  "gene_name": "Fasciculation and elongation protein zeta-2",
  "gene_symbol": "FEZ2",
  "term_id": "UNKNOWN:0001"
}